secondary piRNA processing [GO:0140965] (biological process) References: PMID:29281264, PMID:32895365 Relationships: is a type of GO:0034587 Definition: A process leading to the generation of a functional secondary piRNA, involving a self-perpetuating piRNA loop, often called the ping-pong cycle, in which piRNAs are amplified by pairing with complementary transcripts (for example the transposable element mRNA target). In Drosophila, the processing involves the piwi proteins aubergine and Argonaute 3 and in mice, the piwi proteins Piwil2 and Piwil4. Also known as: ping-pong derived piRNA, secondary PIWI-associated RNA processing, secondary piRNA biogenesis, ping-pong amplification